early phagosome membrane [GO:0036186] (cellular component) Also known as: early phagocytic vesicle membrane Relationships: is a type of phagocytic vesicle membrane [GO:0030670]; is part of GO:0032009 Sources: GOC:phg Definition: The lipid bilayer surrounding an early phagosome.